{
  "gene_name": "Mitochondria-eating protein",
  "gene_symbol": "SPATA18",
  "term_label": "mitochondrial outer membrane",
  "gene": "UniProtKB:Q8TC71",
  "term_id": "GO:0005741"
}